response to oleic acid [GO:0034201] (BP) Definition: Any process that results in a change in state or activity of a cell or an organism (in terms of movement, secretion, enzyme production, gene expression, etc.) as a result of an oleic acid stimulus. Sources: GOC:lp Also known as: response to oleate Relationships: is a type of GO:0070542 Subtypes: GO:0071400